L-tyrosine 2,3-aminomutase activity [GO:0050368] (molecular function) Sources: RHEA:15781 Relationships: is a type of intramolecular aminotransferase activity [GO:0016869] Definition: Catalysis of the reaction: L-tyrosine = 3-amino-3-(4-hydroxyphenyl)propanoate. Also known as: tyrosine 2,3-aminomutase activity, tyrosine alpha,beta-mutase activity